mesenchyme migration [GO:0090131] (biological process) Definition: The process in which the population of cells that make up a mesenchyme undergo directed movement. Sources: GOC:ascb_2009, GOC:dph, GOC:tb Relationships: is_a tissue migration [GO:0090130]; is part of mesenchyme morphogenesis [GO:0072132] Subtypes: mesenchyme migration involved in limb bud formation [GO:0090496]